{
  "gene": "UniProtKB:P20618",
  "gene_symbol": "PSMB1",
  "term_id": "GO:0005737",
  "term_label": "cytoplasm",
  "gene_name": "Proteasome subunit beta type-1"
}